{
  "gene": "UniProtKB:Q9UQM7",
  "term_label": "calmodulin binding",
  "gene_symbol": "CAMK2A",
  "term_id": "GO:0005516",
  "gene_name": "Calcium_calmodulin-dependent protein kinase type II subunit alpha"
}